{
  "term_label": "Unknown molecular function",
  "gene": "UniProtKB:C9JFL3",
  "term_id": "UNKNOWN:0001",
  "gene_symbol": "PHGR1",
  "gene_name": "Proline, histidine and glycine-rich protein 1"
}